{
  "term_id": "GO:0000785",
  "gene_symbol": "SIN3A",
  "gene": "UniProtKB:Q96ST3",
  "gene_name": "Paired amphipathic helix protein Sin3a",
  "term_label": "chromatin"
}